negative regulation of epidermal growth factor receptor signaling pathway involved in heart process [GO:1905283] (biological process) References: PMID:23069713 Sources: GOC:BHF, GOC:BHF_miRNA, GOC:TermGenie, GOC:bc, GO_REF:0000058 Relationships: is a type of GO:0042059; is a type of negative regulation of multicellular organismal process [GO:0051241]; is_a regulation of epidermal growth factor receptor signaling pathway involved in heart process [GO:1905282]; negatively regulates epidermal growth factor receptor signaling pathway involved in heart process [GO:1905251] Definition: Any process that stops, prevents or reduces the frequency, rate or extent of epidermal growth factor receptor signaling pathway involved in heart process. Also known as: down regulation of EGF receptor signaling pathway involved in heart process, down regulation of EGF receptor signalling pathway involved in heart process, down regulation of EGFR signaling pathway involved in heart process, down regulation of ERBB1 signaling pathway involved in heart process, down regulation of epidermal growth factor receptor signaling pathway involved in heart process, down regulation of epidermal growth factor receptor signalling pathway involved in heart process, down regulation of receptor tyrosine-protein kinase erbB-1 signaling pathway involved in heart process, down-regulation of EGF receptor signaling pathway involved in heart process, down-regulation of EGF receptor signalling pathway involved in heart process, down-regulation of EGFR signaling pathway involved in heart process, down-regulation of ERBB1 signaling pathway involved in heart process, down-regulation of epidermal growth factor receptor signaling pathway involved in heart process, down-regulation of epidermal growth factor receptor signalling pathway involved in heart process, down-regulation of receptor tyrosine-protein kinase erbB-1 signaling pathway involved in heart process, downregulation of EGF receptor signaling pathway involved in heart process, downregulation of EGF receptor signalling pathway involved in heart process, downregulation of EGFR signaling pathway involved in heart process, downregulation of ERBB1 signaling pathway involved in heart process, downregulation of epidermal growth factor receptor signaling pathway involved in heart process, downregulation of epidermal growth factor receptor signalling pathway involved in heart process, downregulation of receptor tyrosine-protein kinase erbB-1 signaling pathway involved in heart process, negative regulation of EGF receptor signaling pathway involved in heart process, negative regulation of EGF receptor signalling pathway involved in heart process, negative regulation of EGFR signaling pathway involved in heart process, negative regulation of ERBB1 signaling pathway involved in heart process, negative regulation of epidermal growth factor receptor signalling pathway involved in heart process, negative regulation of receptor tyrosine-protein kinase erbB-1 signaling pathway involved in heart process, inhibition of EGF receptor signaling pathway involved in heart process, inhibition of EGF receptor signalling pathway involved in heart process, inhibition of EGFR signaling pathway involved in heart process, inhibition of ERBB1 signaling pathway involved in heart process, inhibition of epidermal growth factor receptor signaling pathway involved in heart process, inhibition of epidermal growth factor receptor signalling pathway involved in heart process, inhibition of receptor tyrosine-protein kinase erbB-1 signaling pathway involved in heart process, down regulation of EGF receptor signaling pathway involved in cardiac process, down regulation of EGF receptor signalling pathway involved in cardiac process, down regulation of EGFR signaling pathway involved in cardiac process, down regulation of ERBB1 signaling pathway involved in cardiac process, down regulation of epidermal growth factor receptor signaling pathway involved in cardiac process, down regulation of epidermal growth factor receptor signalling pathway involved in cardiac process, down regulation of receptor tyrosine-protein kinase erbB-1 signaling pathway involved in cardiac process, down-regulation of EGF receptor signaling pathway involved in cardiac process, down-regulation of EGF receptor signalling pathway involved in cardiac process, down-regulation of EGFR signaling pathway involved in cardiac process, down-regulation of ERBB1 signaling pathway involved in cardiac process, down-regulation of epidermal growth factor receptor signaling pathway involved in cardiac process, down-regulation of epidermal growth factor receptor signalling pathway involved in cardiac process, down-regulation of receptor tyrosine-protein kinase erbB-1 signaling pathway involved in cardiac process, downregulation of EGF receptor signaling pathway involved in cardiac process, downregulation of EGF receptor signalling pathway involved in cardiac process, downregulation of EGFR signaling pathway involved in cardiac process, downregulation of ERBB1 signaling pathway involved in cardiac process, downregulation of epidermal growth factor receptor signaling pathway involved in cardiac process, downregulation of epidermal growth factor receptor signalling pathway involved in cardiac process, downregulation of receptor tyrosine-protein kinase erbB-1 signaling pathway involved in cardiac process, inhibition of EGF receptor signaling pathway involved in cardiac process, inhibition of EGF receptor signalling pathway involved in cardiac process, inhibition of EGFR signaling pathway involved in cardiac process, inhibition of ERBB1 signaling pathway involved in cardiac process, inhibition of epidermal growth factor receptor signaling pathway involved in cardiac process, inhibition of epidermal growth factor receptor signalling pathway involved in cardiac process, inhibition of receptor tyrosine-protein kinase erbB-1 signaling pathway involved in cardiac process, negative regulation of EGF receptor signaling pathway involved in cardiac process, negative regulation of EGF receptor signalling pathway involved in cardiac process, negative regulation of EGFR signaling pathway involved in cardiac process, negative regulation of ERBB1 signaling pathway involved in cardiac process, negative regulation of epidermal growth factor receptor signaling pathway involved in cardiac process, negative regulation of epidermal growth factor receptor signalling pathway involved in cardiac process, negative regulation of receptor tyrosine-protein kinase erbB-1 signaling pathway involved in cardiac process